formate biosynthetic process [GO:0015943] (biological process) Definition: The chemical reactions and pathways resulting in the formation of formate, also known as methanoate, the anion HCOO- derived from methanoic (formic) acid. Relationships: is a type of GO:0015942; is a type of GO:0072330 Also known as: formate anabolism, formate biosynthesis, formate formation, formate synthesis, formic acid biosynthesis, formic acid biosynthetic process Sources: ISBN:0198506732